nonphotochemical quenching [GO:0010196] (BP) References: PMID:10667783, PMID:10938857 Definition: The process by which excess light energy absorbed by chlorophyll and not used to drive photosynthesis is emitted as heat. This process helps maintain the balance between dissipation and utilization of light energy to minimize generation of oxidizing molecules, thereby protecting the plant against photo-oxidative damage. Relationships: is a type of GO:1990066